{
  "gene_name": "D(1A) dopamine receptor",
  "term_label": "positive regulation of MAPK cascade",
  "gene": "UniProtKB:P21728",
  "gene_symbol": "DRD1",
  "term_id": "GO:0043410"
}